{
  "term_label": "potassium:proton antiporter activity",
  "gene": "UniProtKB:Q96T83",
  "gene_symbol": "SLC9A7",
  "term_id": "GO:0015386",
  "gene_name": "Sodium_hydrogen exchanger 7"
}